{
  "gene_symbol": "C1QL2",
  "term_id": "GO:0005615",
  "gene_name": "Complement C1q-like protein 2",
  "term_label": "extracellular space",
  "gene": "UniProtKB:Q7Z5L3"
}